{
  "term_label": "regulation of transcription by RNA polymerase II",
  "term_id": "GO:0006357",
  "gene": "UniProtKB:Q13398",
  "gene_name": "Zinc finger protein 211",
  "gene_symbol": "ZNF211"
}